{
  "term_id": "GO:0003729",
  "term_label": "mRNA binding",
  "gene": "UniProtKB:Q8WW36",
  "gene_symbol": "ZCCHC13",
  "gene_name": "Zinc finger CCHC domain-containing protein 13"
}